{
  "gene": "UniProtKB:P38936",
  "term_label": "nucleus",
  "gene_name": "Cyclin-dependent kinase inhibitor 1",
  "gene_symbol": "CDKN1A",
  "term_id": "GO:0005634"
}